regulation of RIG-I signaling pathway [GO:0039535] (biological process) Sources: GOC:bf, GOC:jl Relationships: is a type of regulation of cytoplasmic pattern recognition receptor signaling pathway [GO:0039531]; regulates RIG-I signaling pathway [GO:0039529] Subtypes: negative regulation of RIG-I signaling pathway [GO:0039536], positive regulation of RIG-I signaling pathway [GO:1900246] Also known as: regulation of DDX58 signaling pathway, regulation of RIG-I signalling pathway, regulation of retinoic acid inducible gene I signaling pathway Definition: Any process that modulates the frequency, rate or extent of the RIG-I signaling pathway.